{
  "gene": "UniProtKB:Q9Y698",
  "term_label": "channel regulator activity",
  "gene_name": "Voltage-dependent calcium channel gamma-2 subunit",
  "term_id": "GO:0016247",
  "gene_symbol": "CACNG2"
}